{
  "gene_symbol": "TMEM14A",
  "gene_name": "Transmembrane protein 14A",
  "term_id": "UNKNOWN:0001",
  "term_label": "Unknown molecular function",
  "gene": "UniProtKB:Q9Y6G1"
}